{
  "gene": "UniProtKB:Q3SY77",
  "term_label": "Unknown biological process",
  "gene_name": "UDP-glucuronosyltransferase 3A2",
  "term_id": "UNKNOWN:0002",
  "gene_symbol": "UGT3A2"
}